stromal side of plastid thylakoid membrane [GO:0098572] (cellular component) Definition: The side (leaflet) of the plastid thylakoid membrane that faces the stroma, and any proteins embedded in it or loosely bound to its surface. Sources: GOC:dos Relationships: is a type of side of membrane [GO:0098552]; is part of plastid thylakoid membrane [GO:0055035]